{
  "gene_name": "Histone deacetylase 6",
  "term_id": "GO:0005737",
  "gene": "UniProtKB:Q9UBN7",
  "gene_symbol": "HDAC6",
  "term_label": "cytoplasm"
}